positive regulation of branching involved in ureteric bud morphogenesis [GO:0090190] (biological process) Sources: GOC:dph, GOC:tb, GOC:yaf Definition: Any process that increases the rate, frequency or extent of branching involved in ureteric bud morphogenesis, the process in which the branching structure of the ureteric bud is generated and organized. The ureteric bud is an epithelial tube that grows out from the metanephric duct. The bud elongates and branches to give rise to the ureter and kidney collecting tubules. Relationships: is a type of positive regulation of multicellular organismal process [GO:0051240]; is a type of GO:0090189; is_a positive regulation of morphogenesis of an epithelium [GO:1905332]; positively regulates GO:0001658